{
  "gene_name": "Guanine nucleotide-binding protein G(I)_G(S)_G(T) subunit beta-2",
  "term_id": "GO:0030159",
  "term_label": "signaling receptor complex adaptor activity",
  "gene": "UniProtKB:P62879",
  "gene_symbol": "GNB2"
}